regulation of double fertilization forming a zygote and endosperm [GO:0080155] (biological process) Relationships: is a type of GO:0080154; regulates GO:0009567 References: PMID:20478994 Sources: GOC:DHL Definition: Any process that modulates the rate, frequency or extent of double fertilization forming a zygote and endosperm. Double fertilization forming a zygote and endosperm is a type of fertilization where one of the two sperm nuclei from the pollen tube fuses with the egg nucleus to form a 2n zygote, and the other fuses with the two polar nuclei to form the 3n primary endosperm nucleus and then develops into the endosperm. The ploidy level of the 2n zygote and 3n primary endosperm nucleus is determined by the ploidy level of the parents involved. An example of this component is found in Arabidopsis thaliana. Subtypes: prevention of polyspermy during double fertilization [GO:0160071]